{
  "gene_name": "Thioredoxin-like protein 4A",
  "gene_symbol": "TXNL4A",
  "term_id": "UNKNOWN:0001",
  "gene": "UniProtKB:P83876",
  "term_label": "Unknown molecular function"
}